{
  "term_label": "Unknown cellular component",
  "gene_name": "Mucin-3B",
  "gene": "UniProtKB:Q9H195",
  "gene_symbol": "MUC3B",
  "term_id": "UNKNOWN:0003"
}